{
  "gene": "UniProtKB:Q8N6I1",
  "term_label": "transcription corepressor activity",
  "gene_name": "EP300-interacting inhibitor of differentiation 2",
  "gene_symbol": "EID2",
  "term_id": "GO:0003714"
}